{
  "gene_symbol": "STUB1",
  "gene_name": "E3 ubiquitin-protein ligase CHIP",
  "gene": "UniProtKB:Q9UNE7",
  "term_id": "GO:0043161",
  "term_label": "proteasome-mediated ubiquitin-dependent protein catabolic process"
}